{
  "term_id": "GO:0019346",
  "gene": "UniProtKB:P32929",
  "gene_name": "Cystathionine gamma-lyase",
  "term_label": "transsulfuration",
  "gene_symbol": "CTH"
}